negative regulation of bone remodeling [GO:0046851] (biological process) Sources: GOC:ai Also known as: down regulation of bone remodeling, down-regulation of bone remodeling, downregulation of bone remodeling, negative regulation of bone remodelling, inhibition of bone remodeling Subtypes: negative regulation of bone resorption [GO:0045779] Definition: Any process that stops, prevents, or reduces the frequency, rate or extent of bone remodeling. Relationships: is a type of GO:0034104; is a type of GO:0046850; negatively regulates bone remodeling [GO:0046849]